{
  "gene_name": "CDKN2AIP N-terminal-like protein",
  "term_label": "Unknown cellular component",
  "gene": "UniProtKB:Q96HQ2",
  "gene_symbol": "CDKN2AIPNL",
  "term_id": "UNKNOWN:0003"
}